{
  "term_id": "GO:0005886",
  "gene": "UniProtKB:O00220",
  "gene_name": "Tumor necrosis factor receptor superfamily member 10A",
  "gene_symbol": "TNFRSF10A",
  "term_label": "plasma membrane"
}